{
  "term_id": "GO:0005829",
  "gene_symbol": "RABIF",
  "gene_name": "Guanine nucleotide exchange factor MSS4",
  "gene": "UniProtKB:P47224",
  "term_label": "cytosol"
}